{
  "gene": "UniProtKB:Q8IW41",
  "gene_name": "MAP kinase-activated protein kinase 5",
  "term_label": "mitogen-activated protein kinase binding",
  "term_id": "GO:0051019",
  "gene_symbol": "MAPKAPK5"
}